leaflet morphogenesis [GO:0060794] (biological process) Definition: The process in which the anatomical structures of the leaflet are generated and organized. Subtypes: primary leaflet morphogenesis [GO:0060778], secondary leaflet morphogenesis [GO:0060779], intercalary leaflet morphogenesis [GO:0060780] Sources: GOC:dph, GOC:sdb_2009, GOC:tb Relationships: is a type of GO:0009653; BFO_0000050 GO:0060777